{
  "gene_name": "Nuclear envelope pore membrane protein POM 121",
  "gene": "UniProtKB:Q96HA1",
  "gene_symbol": "POM121",
  "term_label": "nuclear pore",
  "term_id": "GO:0005643"
}